{
  "term_id": "GO:0005634",
  "gene": "UniProtKB:Q9NTI5",
  "gene_name": "Sister chromatid cohesion protein PDS5 homolog B",
  "term_label": "nucleus",
  "gene_symbol": "PDS5B"
}